{
  "gene": "UniProtKB:Q3B8N2",
  "gene_name": "Galectin-9B",
  "term_label": "positive regulation of gene expression",
  "gene_symbol": "LGALS9B",
  "term_id": "GO:0010628"
}